meiotic recombination checkpoint signaling [GO:0051598] (biological process) Also known as: meiotic recombination checkpoint, pachytene checkpoint, signal transduction involved in meiotic recombination checkpoint References: PMID:14718568 Relationships: is a type of meiotic cell cycle checkpoint signaling [GO:0033313]; is a type of negative regulation of meiotic nuclear division [GO:0045835] Definition: A signaling process that contributes to a meiotic recombination checkpoint, that acts during late prophase I (pachytene) and prevents segregation of homologous chromosomes until recombination is completed, ensuring proper distribution of the genetic material to the gametes.